{
  "term_id": "GO:0061608",
  "term_label": "nuclear import signal receptor activity",
  "gene": "UniProtKB:O60684",
  "gene_symbol": "KPNA6",
  "gene_name": "Importin subunit alpha-7"
}